{
  "term_id": "GO:0043410",
  "gene_name": "Insulin-like growth factor 1 receptor",
  "gene_symbol": "IGF1R",
  "gene": "UniProtKB:P08069",
  "term_label": "positive regulation of MAPK cascade"
}